{
  "gene_symbol": "A0A0G2JQF1",
  "gene_name": "Uncharacterized protein",
  "gene": "UniProtKB:A0A0G2JQF1",
  "term_id": "UNKNOWN:0002",
  "term_label": "Unknown biological process"
}